viral intermediate capsid [GO:0039626] (cellular component) Relationships: is a type of virion component [GO:0044423]; is part of GO:0019030 Sources: UniProtKB-KW:KW-1154 Definition: The intermediate layer of a triple concentric icosahedral capsid. Intermediate capsids are part of reoviridae virions. Also known as: intermediate capsid